{
  "gene": "UniProtKB:Q5VT03",
  "term_label": "Unknown molecular function",
  "term_id": "UNKNOWN:0001",
  "gene_symbol": "NUTM2D",
  "gene_name": "NUT family member 2D"
}